{
  "gene_name": "Zinc finger protein 878",
  "gene_symbol": "ZNF878",
  "term_id": "GO:0000981",
  "term_label": "DNA-binding transcription factor activity, RNA polymerase II-specific",
  "gene": "UniProtKB:C9JN71"
}